diacetylchitobiose metabolic process [GO:0052778] (biological process) Definition: The chemical reactions and pathways involving diacetylchitobiose, the N,N'-diacetylated derivative of chitobiose. Relationships: is a type of carbohydrate derivative metabolic process [GO:1901135] Subtypes: diacetylchitobiose catabolic process [GO:0052777] References: PMID:22797760 Also known as: diacetylchitobiose metabolism